adenosine-phosphate deaminase activity [GO:0047623] (molecular function) Relationships: is a type of hydrolase activity, acting on carbon-nitrogen (but not peptide) bonds, in cyclic amidines [GO:0016814]; is a type of deaminase activity [GO:0019239] Also known as: adenine nucleotide deaminase activity, adenosine (phosphate) deaminase activity, adenosine-phosphate aminohydrolase activity Sources: EC:3.5.4.17 Definition: Catalysis of the reaction: an adenosine-phosphate + H20 = an inosine phosphate + NH3. Catalyzes the deamination of AMP, ADP or ATP. Subtypes: GO:0003876, GO:0047629, ATP deaminase activity [GO:0047692] Note: Consider instead annotating to one of the more specific terms: AMP deaminase activity ; GO:0003876, ADP deaminase activity ; GO:0047629, or ATP deaminase activity ; GO:0047692.